{
  "term_label": "Unknown molecular function",
  "gene": "UniProtKB:Q68CZ6",
  "gene_name": "HAUS augmin-like complex subunit 3",
  "gene_symbol": "HAUS3",
  "term_id": "UNKNOWN:0001"
}